{
  "gene_symbol": "VCAN",
  "gene_name": "Versican core protein",
  "term_label": "skeletal system development",
  "gene": "UniProtKB:P13611",
  "term_id": "GO:0001501"
}